{
  "gene_name": "Dihydrolipoyllysine-residue succinyltransferase component of 2-oxoglutarate dehydrogenase complex, mitochondrial",
  "gene_symbol": "DLST",
  "term_label": "mitochondrion",
  "gene": "UniProtKB:P36957",
  "term_id": "GO:0005739"
}